{
  "term_label": "plasma membrane",
  "gene_name": "Adhesion G protein-coupled receptor G3",
  "gene": "UniProtKB:Q86Y34",
  "gene_symbol": "ADGRG3",
  "term_id": "GO:0005886"
}